{
  "term_id": "GO:0019185",
  "gene": "UniProtKB:Q5SXM2",
  "gene_symbol": "SNAPC4",
  "term_label": "snRNA-activating protein complex",
  "gene_name": "snRNA-activating protein complex subunit 4"
}